{
  "gene": "UniProtKB:P48739",
  "term_label": "phosphatidylinositol binding",
  "term_id": "GO:0035091",
  "gene_name": "Phosphatidylinositol transfer protein beta isoform",
  "gene_symbol": "PITPNB"
}